{
  "gene": "UniProtKB:P50281",
  "gene_symbol": "MMP14",
  "term_id": "GO:0005615",
  "term_label": "extracellular space",
  "gene_name": "Matrix metalloproteinase-14"
}